positive regulation of cellular response to oxidopamine [GO:1905848] (biological process) Relationships: is_a GO:0048522; is a type of positive regulation of response to stimulus [GO:0048584]; is a type of regulation of cellular response to oxidopamine [GO:1905846]; positively regulates cellular response to oxidopamine [GO:1905842] Also known as: up regulation of cellular response to oxidopamine, up-regulation of cellular response to oxidopamine, upregulation of cellular response to oxidopamine, activation of cellular response to oxidopamine References: PMID:23721876 Sources: GOC:TermGenie, GO_REF:0000058 Definition: Any process that activates or increases the frequency, rate or extent of cellular response to oxidopamine.